tricyclene synthase activity [GO:0102701] (MF) Definition: Catalysis of the reaction: geranyl diphosphate(3-) = tricyclene + diphosphoric acid. Sources: EC:4.2.3.105, GOC:pz Relationships: is_a carbon-oxygen lyase activity, acting on phosphates [GO:0016838]